xylem vessel member cell differentiation [GO:0048759] (biological process) Also known as: vessel element cell differentiation, vessel member cell differentiation Sources: GOC:jid, PO:0002003 Relationships: is a type of tracheary element differentiation [GO:1905177]; is part of GO:0010089 Definition: The process in which a relatively unspecialized cell acquires specialized features of a vessel member cell. A vessel member cell is one of the components of a vessel in the xylem. It is a dead cell with the wall between adjacent members being variously perforated and the walls that persist variously thickened.